{
  "term_id": "GO:0007080",
  "term_label": "mitotic metaphase chromosome alignment",
  "gene": "UniProtKB:Q8N9V6",
  "gene_name": "Ankyrin repeat domain-containing protein 53",
  "gene_symbol": "ANKRD53"
}